{
  "gene_symbol": "BRCA2",
  "term_label": "single-stranded DNA binding",
  "gene_name": "Breast cancer type 2 susceptibility protein",
  "gene": "UniProtKB:P51587",
  "term_id": "GO:0003697"
}